cell wall disassembly [GO:0044277] (BP) Relationships: is a type of GO:0022411; is a type of cell wall organization [GO:0071555] Definition: A process that results in the breakdown of the cell wall. Also known as: cellular cell wall disassembly Sources: GOC:jl Subtypes: GO:0009830, fungal-type cell wall disassembly [GO:0071853]